{
  "gene": "UniProtKB:P14555",
  "term_id": "GO:0042130",
  "gene_symbol": "PLA2G2A",
  "term_label": "negative regulation of T cell proliferation",
  "gene_name": "Phospholipase A2, membrane associated"
}